{
  "gene_symbol": "TRIM10",
  "term_label": "innate immune response",
  "gene_name": "Tripartite motif-containing protein 10",
  "term_id": "GO:0045087",
  "gene": "UniProtKB:Q9UDY6"
}